1-phosphatidyl-1D-myo-inositol 3,5-bisphosphate biosynthetic process [GO:1903102] (biological process) Also known as: 1-phosphatidyl-1D-myo-inositol 3,5-bisphosphate anabolism, 1-phosphatidyl-1D-myo-inositol 3,5-bisphosphate biosynthesis, 1-phosphatidyl-1D-myo-inositol 3,5-bisphosphate formation, 1-phosphatidyl-1D-myo-inositol 3,5-bisphosphate synthesis Definition: The chemical reactions and pathways resulting in the formation of 1-phosphatidyl-1D-myo-inositol 3,5-bisphosphate. References: PMID:19037259 Sources: GOC:TermGenie, GOC:bhm, GO_REF:0000068 Relationships: is a type of phosphatidylinositol phosphate biosynthetic process [GO:0046854]; is a type of 1-phosphatidyl-1D-myo-inositol 3,5-bisphosphate metabolic process [GO:1903100]